{
  "gene_symbol": "ADA",
  "term_label": "adenosine catabolic process",
  "gene": "UniProtKB:P00813",
  "gene_name": "Adenosine deaminase",
  "term_id": "GO:0006154"
}